{
  "gene_symbol": "SYT6",
  "term_label": "exocytic vesicle",
  "gene_name": "Synaptotagmin-6",
  "gene": "UniProtKB:Q5T7P8",
  "term_id": "GO:0070382"
}